{
  "gene_name": "Nucleosome assembly protein 1-like 1",
  "gene": "UniProtKB:P55209",
  "gene_symbol": "NAP1L1",
  "term_id": "GO:0005634",
  "term_label": "nucleus"
}